{
  "term_id": "GO:0005085",
  "gene_symbol": "FARP2",
  "gene": "UniProtKB:O94887",
  "gene_name": "FERM, ARHGEF and pleckstrin domain-containing protein 2",
  "term_label": "guanyl-nucleotide exchange factor activity"
}